{
  "term_id": "GO:0050877",
  "gene_name": "AF4_FMR2 family member 3",
  "term_label": "nervous system process",
  "gene": "UniProtKB:P51826",
  "gene_symbol": "AFF3"
}